{
  "gene_symbol": "SPSB2",
  "term_id": "GO:0019005",
  "gene_name": "SPRY domain-containing SOCS box protein 2",
  "term_label": "SCF ubiquitin ligase complex",
  "gene": "UniProtKB:Q99619"
}